{
  "term_id": "GO:0007160",
  "term_label": "cell-matrix adhesion",
  "gene": "UniProtKB:Q7RTW8",
  "gene_name": "Otoancorin",
  "gene_symbol": "OTOA"
}